{
  "gene_name": "Tubulin alpha-1B chain",
  "term_label": "cytoplasm",
  "gene_symbol": "TUBA1B",
  "term_id": "GO:0005737",
  "gene": "UniProtKB:P68363"
}